cobalt ion transport [GO:0006824] (biological process) Sources: GOC:ai Definition: The directed movement of cobalt (Co2+) ions into, out of or within a cell, or between cells, by means of some agent such as a transporter or pore. Relationships: is a type of transition metal ion transport [GO:0000041]; is a type of monoatomic cation transmembrane transport [GO:0098655] Also known as: cobalt transport